vestibular receptor cell fate commitment [GO:0060115] (biological process) Relationships: is a type of GO:0060120; is part of GO:0060114 Sources: GOC:dph Also known as: vestibular hair cell fate commitment Definition: The process in which a cell becomes committed to become a vestibular receptor cell.